2-hydroxyglutarate synthase activity [GO:0019142] (molecular function) Definition: Catalysis of the reaction: glyoxylate + H2O + propanoyl-CoA = 2-hydroxyglutarate + CoA + H+. Also known as: 2-hydroxyglutarate glyoxylate-lyase (CoA-propanoylating) activity, 2-hydroxyglutaratic synthetase activity, 2-hydroxyglutaric synthetase activity, alpha-hydroxyglutarate synthase activity, hydroxyglutarate synthase activity, propanoyl-CoA:glyoxylate C-propanoyltransferase (thioester-hydrolysing, 2-carboxyethyl-forming) Sources: RHEA:19185 Relationships: is a type of acyltransferase activity, acyl groups converted into alkyl on transfer [GO:0046912]